{
  "gene_symbol": "ZFAND2B",
  "gene": "UniProtKB:Q8WV99",
  "term_id": "GO:0005783",
  "term_label": "endoplasmic reticulum",
  "gene_name": "AN1-type zinc finger protein 2B"
}